{
  "gene": "UniProtKB:Q9Y333",
  "term_id": "GO:1990726",
  "gene_name": "U6 snRNA-associated Sm-like protein LSm2",
  "term_label": "Lsm1-7-Pat1 complex",
  "gene_symbol": "LSM2"
}